{
  "term_id": "GO:0043005",
  "gene_name": "Calcium_calmodulin-dependent protein kinase type II subunit gamma",
  "gene_symbol": "CAMK2G",
  "gene": "UniProtKB:Q13555",
  "term_label": "neuron projection"
}